{
  "gene_symbol": "TBC1D5",
  "gene": "UniProtKB:Q92609",
  "term_label": "retrograde transport, endosome to Golgi",
  "term_id": "GO:0042147",
  "gene_name": "TBC1 domain family member 5"
}